{
  "term_id": "UNKNOWN:0001",
  "gene": "UniProtKB:Q96KT7",
  "term_label": "Unknown molecular function",
  "gene_symbol": "SLC35G5",
  "gene_name": "Solute carrier family 35 member G5"
}